fructose metabolic process [GO:0006000] (biological process) Subtypes: fructose catabolic process [GO:0006001], GO:0046370 Relationships: is a type of hexose metabolic process [GO:0019318] Also known as: fructose metabolism Sources: ISBN:0198506732 Definition: The chemical reactions and pathways involving fructose, the ketohexose arabino-2-hexulose. Fructose exists in a open chain form or as a ring compound. D-fructose is the sweetest of the sugars and is found free in a large number of fruits and honey.